{
  "term_id": "GO:0004984",
  "term_label": "olfactory receptor activity",
  "gene_name": "Olfactory receptor 2M3",
  "gene": "UniProtKB:Q8NG83",
  "gene_symbol": "OR2M3"
}